{
  "term_id": "GO:0000978",
  "gene_name": "Nuclear receptor subfamily 4 group A member 2",
  "gene": "UniProtKB:P43354",
  "gene_symbol": "NR4A2",
  "term_label": "RNA polymerase II cis-regulatory region sequence-specific DNA binding"
}